{
  "gene_name": "UDP-glucuronosyltransferase 2A1",
  "term_id": "GO:0015020",
  "gene_symbol": "UGT2A1",
  "gene": "UniProtKB:P0DTE4",
  "term_label": "glucuronosyltransferase activity"
}